{
  "gene_symbol": "DERL1",
  "term_id": "GO:0036503",
  "gene": "UniProtKB:Q9BUN8",
  "term_label": "ERAD pathway",
  "gene_name": "Derlin-1"
}